{
  "gene_symbol": "DSCAML1",
  "gene": "UniProtKB:Q8TD84",
  "term_id": "GO:0007417",
  "term_label": "central nervous system development",
  "gene_name": "Cell adhesion molecule DSCAML1"
}